{
  "term_id": "GO:0006357",
  "term_label": "regulation of transcription by RNA polymerase II",
  "gene": "UniProtKB:Q8IYA7",
  "gene_symbol": "MKX",
  "gene_name": "Homeobox protein Mohawk"
}